{
  "term_label": "cilium assembly",
  "term_id": "GO:0060271",
  "gene_name": "C2 domain-containing protein 3",
  "gene": "UniProtKB:Q4AC94",
  "gene_symbol": "C2CD3"
}